embryonic ectodermal digestive tract morphogenesis [GO:0048613] (biological process) Also known as: embryonic ectodermal gut morphogenesis Definition: The process, occurring during the embryonic phase, by which the anatomical structures of the ectodermal digestive tract are generated and organized. Sources: GOC:jid, GOC:rc Relationships: is a type of embryonic morphogenesis [GO:0048598]; is part of embryonic digestive tract morphogenesis [GO:0048557]; is part of ectodermal digestive tract morphogenesis [GO:0048567]; is part of GO:0048611